{
  "gene_symbol": "OSBPL11",
  "term_label": "cytosol",
  "term_id": "GO:0005829",
  "gene": "UniProtKB:Q9BXB4",
  "gene_name": "Oxysterol-binding protein-related protein 11"
}